exocytic vesicle [GO:0070382] (cellular component) Also known as: exocytic constitutive secretory pathway transport vesicle, exocytotic vesicle Subtypes: synaptic vesicle [GO:0008021], Golgi to plasma membrane transport vesicle [GO:0070319], endosome to plasma membrane transport vesicle [GO:0070381] Relationships: is a type of GO:0030133; is_a GO:0099503 Sources: GOC:kad, GOC:mah Definition: A transport vesicle that mediates transport from an intracellular compartment to the plasma membrane, and fuses with the plasma membrane to release various cargo molecules, such as proteins or hormones, by exocytosis.